{
  "term_id": "GO:0005634",
  "gene_symbol": "SETSIP",
  "gene_name": "Protein SETSIP",
  "term_label": "nucleus",
  "gene": "UniProtKB:P0DME0"
}